{
  "gene": "UniProtKB:O94830",
  "gene_name": "Phospholipase DDHD2",
  "term_label": "Unknown biological process",
  "term_id": "UNKNOWN:0002",
  "gene_symbol": "DDHD2"
}